{
  "term_id": "GO:0005871",
  "gene": "UniProtKB:Q9NQT8",
  "gene_symbol": "KIF13B",
  "term_label": "kinesin complex",
  "gene_name": "Kinesin-like protein KIF13B"
}